{
  "gene_name": "RING finger protein 32",
  "gene": "UniProtKB:Q9H0A6",
  "gene_symbol": "RNF32",
  "term_id": "UNKNOWN:0003",
  "term_label": "Unknown cellular component"
}